{
  "gene_symbol": "OXLD1",
  "gene": "UniProtKB:Q5BKU9",
  "term_label": "Unknown molecular function",
  "term_id": "UNKNOWN:0001",
  "gene_name": "Oxidoreductase-like domain-containing protein 1"
}